cellular response to potassium ion starvation [GO:0051365] (biological process) Sources: GOC:sm Relationships: is a type of cellular response to starvation [GO:0009267] Definition: Any process that results in a change in state or activity of a cell (in terms of movement, secretion, enzyme production, gene expression, etc.) as a result of deprivation of potassium ions. Also known as: cellular response to K+ ion deprivation, cellular response to K+ ion starvation, cellular response to potassium ion deprivation, cellular response to potassium starvation